neutrophil dispersal [GO:0140635] (biological process) Relationships: is a type of neutrophil migration [GO:1990266] Definition: The movement of a neutrophil away from the site of wound or infection following its initial migration to the site. References: PMID:31727891